lysolecithin acylmutase activity [GO:0050070] (molecular function) Sources: EC:5.4.1.1, RHEA:24356 Relationships: is a type of GO:0016867 Definition: Catalysis of the reaction: 1-acyl-sn-glycero-3-phosphocholine = 2-acyl-sn-glycero-3-phosphocholine. Also known as: lysolecithin 2,3-acylmutase activity, lysolecithin migratase activity